{
  "term_label": "mitochondrion",
  "gene": "UniProtKB:Q9NZJ6",
  "gene_name": "Ubiquinone biosynthesis O-methyltransferase, mitochondrial",
  "gene_symbol": "COQ3",
  "term_id": "GO:0005739"
}